response to viscosity [GO:0097714] (biological process) References: PMID:7061416 Sources: GOC:sl Relationships: is a type of GO:0009628 Subtypes: cellular response to viscosity [GO:0097715] Definition: Any process that results in a change in state or activity of a cell or an organism (in terms of movement, secretion, enzyme production, gene expression, etc.) as a result of a viscosity stimulus.